{
  "term_id": "UNKNOWN:0001",
  "gene_name": "Putative uncharacterized protein MGC163334",
  "gene": "UniProtKB:Q5W150",
  "term_label": "Unknown molecular function",
  "gene_symbol": "Q5W150"
}